chemorepulsion of serotonergic neuron axon [GO:0036519] (biological process) Also known as: chemorepulsion of 5-HT axon, chemorepulsion of serotonergic axon Relationships: is a type of chemorepulsion of axon [GO:0061643]; is part of serotonergic neuron axon guidance [GO:0036515] References: PMID:21106844 Sources: CL:0000850, GOC:PARL, GOC:bf Definition: The process in which a serotonergic neuron growth cone is directed to a specific target site in response to a repulsive chemical cue.